{
  "gene_symbol": "CHMP6",
  "term_label": "nuclear envelope",
  "term_id": "GO:0005635",
  "gene": "UniProtKB:Q96FZ7",
  "gene_name": "Charged multivesicular body protein 6"
}